relaxation of smooth muscle [GO:0044557] (biological process) Also known as: smooth muscle relaxation Subtypes: GO:0044558, GO:0060085, relaxation of vascular associated smooth muscle [GO:0060087] Regulation: regulated by regulation of relaxation of smooth muscle [GO:1901080]; negatively regulated by negative regulation of relaxation of smooth muscle [GO:1901081]; positively regulated by positive regulation of relaxation of smooth muscle [GO:1901082] Definition: A process in which the extent of smooth muscle contraction is reduced. Smooth muscle differs from striated muscle in the much higher actin/myosin ratio, the absence of conspicuous sarcomeres and the ability to contract to a much smaller fraction of its resting length. Sources: GOC:jl Relationships: is a type of relaxation of muscle [GO:0090075]